3-keto-sphinganine metabolic process [GO:0006666] (biological process) Definition: The chemical reactions and pathways involving 3-keto-sphinganine, a derivative of sphinganine with a ketone group at C3. It is an intermediate in the synthesis of sphingosine. Sources: GOC:ai Relationships: is a type of ketone metabolic process [GO:0042180]; is_a sphingoid metabolic process [GO:0046519] Also known as: 3-keto-dihydrosphingosine metabolic process, 3-keto-dihydrosphingosine metabolism, 3-keto-sphinganine metabolism